{
  "gene_name": "Olfactory receptor 1C1",
  "term_label": "signal transduction",
  "term_id": "GO:0007165",
  "gene": "UniProtKB:Q15619",
  "gene_symbol": "OR1C1"
}